{
  "term_label": "mRNA splicing, via spliceosome",
  "gene_name": "U2 small nuclear ribonucleoprotein B''",
  "term_id": "GO:0000398",
  "gene": "UniProtKB:P08579",
  "gene_symbol": "SNRPB2"
}